{
  "gene_symbol": "BARD1",
  "gene_name": "BRCA1-associated RING domain protein 1",
  "term_label": "BRCA1-A complex",
  "term_id": "GO:0070531",
  "gene": "UniProtKB:Q99728"
}